cholecystokinin receptor binding [GO:0031739] (molecular function) Definition: Binding to a cholecystokinin receptor. Sources: GOC:mah, GOC:nln Subtypes: GO:0031740, type B gastrin/cholecystokinin receptor binding [GO:0031741] Also known as: cholecystokinin receptor ligand Relationships: is_a GO:0071855